{
  "gene_name": "Tyrosyl-DNA phosphodiesterase 1",
  "gene_symbol": "TDP1",
  "gene": "UniProtKB:Q9NUW8",
  "term_id": "GO:0003697",
  "term_label": "single-stranded DNA binding"
}